{
  "term_label": "plasma membrane",
  "term_id": "GO:0005886",
  "gene_name": "N-formyl peptide receptor 3",
  "gene_symbol": "FPR3",
  "gene": "UniProtKB:P25089"
}